{
  "term_label": "Unknown biological process",
  "gene_name": "PI-PLC X domain-containing protein 2",
  "gene_symbol": "PLCXD2",
  "term_id": "UNKNOWN:0002",
  "gene": "UniProtKB:Q0VAA5"
}